maltodextrin phosphorylase activity [GO:0031220] (molecular function) References: PMID:10348846 Sources: RHEA:29691 Definition: Catalysis of the reaction: alpha-maltotetraose + phosphate = alpha-D-glucose 1-phosphate + alpha-maltotriose. Relationships: is a type of 1,4-alpha-oligoglucan phosphorylase activity [GO:0004645]